{
  "term_label": "negative regulation of Wnt signaling pathway",
  "term_id": "GO:0030178",
  "gene_name": "Protein CUSTOS",
  "gene_symbol": "CUSTOS",
  "gene": "UniProtKB:Q96C57"
}